{
  "gene_symbol": "NOTCH3",
  "gene_name": "Neurogenic locus notch homolog protein 3",
  "term_label": "axon guidance",
  "gene": "UniProtKB:Q9UM47",
  "term_id": "GO:0007411"
}